{
  "term_id": "UNKNOWN:0001",
  "term_label": "Unknown molecular function",
  "gene_name": "Keratin-associated protein 17-1",
  "gene": "UniProtKB:Q9BYP8",
  "gene_symbol": "KRTAP17-1"
}